NAD-dependent protein lysine deacetylase activity [GO:0034979] (MF) Definition: Catalysis of the reaction: N(6)-acetyl-L-lysyl-[protein] + NAD+ + H2O = L-lysyl-[protein] + 2''-O-acetyl-ADP-D-ribose + nicotinamide. This reaction transfers an acetyl group from a protein to NAD, producing nicotinamide. Sources: GOC:BHF, GOC:mah, RHEA:43636 Also known as: NAD(+)-dependent protein deacylase, NAD-dependent protein deacetylase activity, protein acetyllysine N-acetyltransferase, protein lysine deacetylase, protein lysine deacylase, NAD(+)-dependent protein deacetylase Relationships: is a type of NAD-dependent protein lysine deacylase activity [GO:0141218] Subtypes: histone deacetylase activity, NAD-dependent [GO:0017136], NAD-dependent protein lysine delactylase activity [GO:0141208]